{
  "gene": "UniProtKB:Q9Y4D2",
  "gene_name": "Diacylglycerol lipase-alpha",
  "term_label": "neurogenesis",
  "term_id": "GO:0022008",
  "gene_symbol": "DAGLA"
}